{
  "gene": "UniProtKB:Q86Y78",
  "term_label": "acetylcholine receptor inhibitor activity",
  "gene_name": "Ly6_PLAUR domain-containing protein 6",
  "gene_symbol": "LYPD6",
  "term_id": "GO:0030550"
}